positive regulation of type III interferon production [GO:0034346] (biological process) Relationships: is a type of positive regulation of cytokine production [GO:0001819]; is a type of regulation of type III interferon production [GO:0034344]; positively regulates type III interferon production [GO:0034343] Also known as: positive regulation of type III IFN production, up regulation of type III interferon production, up-regulation of type III interferon production, upregulation of type III interferon production, activation of type III interferon production, stimulation of type III interferon production Note: Note that IL-28A, IL-28B, and IL-29 are types of interferon-lambda. References: PMID:15546383, PMID:16734557 Sources: GOC:add, ISBN:0126896631 Definition: Any process that activates or increases the frequency, rate, or extent of type III interferon production. Interferon lambda is the only member of the type III interferon found so far.